{
  "gene_name": "B9 domain-containing protein 2",
  "term_label": "Unknown molecular function",
  "gene_symbol": "B9D2",
  "term_id": "UNKNOWN:0001",
  "gene": "UniProtKB:Q9BPU9"
}